D-arginase activity [GO:0047817] (MF) Sources: EC:3.5.3.10, RHEA:12901 Also known as: D-arginine amidinohydrolase activity Definition: Catalysis of the reaction: D-arginine + H2O = D-ornithine + urea. Relationships: is a type of hydrolase activity, acting on carbon-nitrogen (but not peptide) bonds, in linear amidines [GO:0016813]